{
  "term_label": "glycosaminoglycan binding",
  "term_id": "GO:0005539",
  "gene": "UniProtKB:Q03167",
  "gene_name": "Transforming growth factor beta receptor type 3",
  "gene_symbol": "TGFBR3"
}